{
  "gene_symbol": "KRT15",
  "term_label": "structural constituent of skin epidermis",
  "term_id": "GO:0030280",
  "gene": "UniProtKB:P19012",
  "gene_name": "Keratin, type I cytoskeletal 15"
}